{
  "gene": "UniProtKB:Q07973",
  "gene_name": "1,25-dihydroxyvitamin D(3) 24-hydroxylase, mitochondrial",
  "gene_symbol": "CYP24A1",
  "term_id": "UNKNOWN:0003",
  "term_label": "Unknown cellular component"
}